{
  "gene": "UniProtKB:Q15024",
  "term_id": "GO:0016075",
  "gene_name": "Exosome complex component RRP42",
  "term_label": "rRNA catabolic process",
  "gene_symbol": "EXOSC7"
}